{
  "gene": "UniProtKB:P61106",
  "term_id": "GO:0045335",
  "gene_name": "Ras-related protein Rab-14",
  "gene_symbol": "RAB14",
  "term_label": "phagocytic vesicle"
}